{
  "gene_name": "Zinc finger and BTB domain-containing protein 4",
  "gene": "UniProtKB:Q9P1Z0",
  "term_label": "RNA polymerase II cis-regulatory region sequence-specific DNA binding",
  "gene_symbol": "ZBTB4",
  "term_id": "GO:0000978"
}